photoreceptor cell differentiation [GO:0046530] (biological process) Definition: The specialization of organization of a photoreceptor, a cell that responds to incident electromagnetic radiation, particularly visible light. An example of this process is found in Drosophila melanogaster. Relationships: is a type of neuron differentiation [GO:0030182] Sources: GOC:ai, ISBN:0198506732 Subtypes: eye photoreceptor cell differentiation [GO:0001754], ocellus photoreceptor cell differentiation [GO:0042705] Regulation: regulated by regulation of photoreceptor cell differentiation [GO:0046532]; negatively regulated by negative regulation of photoreceptor cell differentiation [GO:0046533]; positively regulated by positive regulation of photoreceptor cell differentiation [GO:0046534]